glycerol-2-phosphatase activity [GO:0047954] (molecular function) Sources: EC:3.1.3.19, RHEA:13105 Relationships: is_a phosphatase activity [GO:0016791] Also known as: 2-glycerophosphatase activity, beta-glycerophosphatase activity, beta-glycerophosphate phosphatase activity, glycerol-2-phosphate phosphohydrolase activity Definition: Catalysis of the reaction: glycerol 2-phosphate + H2O = glycerol + phosphate.